{
  "term_label": "vesicle membrane",
  "term_id": "GO:0012506",
  "gene_name": "Annexin A8",
  "gene": "UniProtKB:P13928",
  "gene_symbol": "ANXA8"
}